{
  "gene": "UniProtKB:P12074",
  "gene_name": "Cytochrome c oxidase subunit 6A1, mitochondrial",
  "term_id": "GO:0045277",
  "gene_symbol": "COX6A1",
  "term_label": "respiratory chain complex IV"
}